{
  "gene": "UniProtKB:Q15672",
  "gene_symbol": "TWIST1",
  "gene_name": "Twist-related protein 1",
  "term_label": "RNA polymerase II transcription regulatory region sequence-specific DNA binding",
  "term_id": "GO:0000977"
}